{
  "gene_name": "Homeobox protein SIX1",
  "term_label": "regulation of transcription by RNA polymerase II",
  "term_id": "GO:0006357",
  "gene": "UniProtKB:Q15475",
  "gene_symbol": "SIX1"
}